{
  "term_label": "Unknown cellular component",
  "gene_name": "Quinone oxidoreductase PIG3",
  "gene_symbol": "TP53I3",
  "term_id": "UNKNOWN:0003",
  "gene": "UniProtKB:Q53FA7"
}